syndecan binding [GO:0045545] (MF) Definition: Binding to syndecan, an integral membrane proteoglycan (250-300 kDa) associated largely with epithelial cells. References: PMID:9355727 Sources: GOC:go_curators Relationships: is a type of proteoglycan binding [GO:0043394]